{
  "gene": "UniProtKB:Q13418",
  "gene_symbol": "ILK",
  "gene_name": "Integrin-linked protein kinase",
  "term_id": "GO:0007229",
  "term_label": "integrin-mediated signaling pathway"
}